germarium-derived cystoblast division [GO:0048142] (biological process) Definition: The four rounds of incomplete mitosis undergone by a cystoblast to form a 16-cell cyst of interconnected cells within a germarium. Within the cyst, one cell differentiates into an oocyte while the rest become nurse cells. An example of this process is found in Drosophila melanogaster. Relationships: is a type of GO:0007282; is part of GO:0030727 References: PMID:11131529 Sources: GOC:jid, GOC:mtg_sensu Also known as: germarium-derived cystoblast cell division